defense response by cell wall thickening [GO:0052482] (biological process) Subtypes: defense response by callose deposition in cell wall [GO:0052544] Sources: GOC:mtg_pamgo_17jul06 Also known as: cell wall thickening during defense response Relationships: is a type of defense response [GO:0006952]; is a type of cellular response to stress [GO:0033554]; is_a cell wall thickening [GO:0052386] Definition: A type of cell wall modification, in which the cell wall is reinforced and made thicker, that occurs as part of the defense response of an organism.